{
  "gene": "UniProtKB:Q7Z5Q5",
  "gene_name": "DNA polymerase nu",
  "gene_symbol": "POLN",
  "term_label": "double-strand break repair",
  "term_id": "GO:0006302"
}